{
  "term_label": "transmembrane transport",
  "gene": "UniProtKB:Q9H222",
  "gene_symbol": "ABCG5",
  "term_id": "GO:0055085",
  "gene_name": "ATP-binding cassette sub-family G member 5"
}